{
  "gene": "UniProtKB:Q86V24",
  "term_label": "plasma membrane",
  "gene_symbol": "ADIPOR2",
  "term_id": "GO:0005886",
  "gene_name": "Adiponectin receptor protein 2"
}